arginine:agmatine antiporter activity [GO:0043862] (molecular function) Definition: Catalysis of the reaction: arginine(out) + agmatine(in) = arginine(in) + agmatine(out). References: PMID:17099215 Sources: GOC:jl Relationships: is a type of amino acid transmembrane transporter activity [GO:0015171]; is a type of antiporter activity [GO:0015297]; is a type of carboxylic acid transmembrane transporter activity [GO:0046943] Also known as: arginine-agmatine antiporter activity, arginine-agmatine exchange transporter activity, arginine/agmatine antiporter activity, AdiC